{
  "term_id": "GO:0022008",
  "gene_name": "Fibroblast growth factor 23",
  "term_label": "neurogenesis",
  "gene_symbol": "FGF23",
  "gene": "UniProtKB:Q9GZV9"
}